{
  "term_id": "GO:0051059",
  "gene_symbol": "BCL10",
  "term_label": "NF-kappaB binding",
  "gene_name": "B-cell lymphoma_leukemia 10",
  "gene": "UniProtKB:O95999"
}